brain segmentation [GO:0035284] (biological process) Relationships: is a type of segmentation [GO:0035282]; is part of GO:0007420; is part of central nervous system segmentation [GO:0035283] Definition: Division of the brain into a series of semi-repetitive parts or segments. Sources: GOC:bf